myosuppressin receptor activity [GO:0035013] (molecular function) Definition: Combining with the peptide myosuppressin to initiate a change in cell activity. Sources: GOC:bf Relationships: is a type of GO:0008528